{
  "gene": "UniProtKB:Q96L91",
  "gene_symbol": "EP400",
  "term_id": "GO:0000812",
  "gene_name": "E1A-binding protein p400",
  "term_label": "Swr1 complex"
}